single-stranded DNA-dependent ATP-dependent DNA helicase complex [GO:0017117] (cellular component) Definition: A protein complex that possesses single-stranded DNA-dependent DNA helicase activity. Sources: GOC:mah Also known as: ssDNA-dependent ATP-dependent DNA helicase complex Relationships: is a type of DNA helicase complex [GO:0033202]